regulation of connective tissue growth factor production [GO:0032643] (BP) Definition: Any process that modulates the frequency, rate, or extent of connective tissue growth factor production. Subtypes: negative regulation of connective tissue growth factor production [GO:0032683], positive regulation of connective tissue growth factor production [GO:0032723] Also known as: regulation of CCN2 production, regulation of CTGF production, regulation of Fisp12 production, regulation of Hcs24 production, regulation of IGFBP8 production, regulation of hypertrophic chondrocyte-specific gene product 24 production, regulation of connective tissue growth factor biosynthetic process Sources: GOC:mah Relationships: is a type of regulation of cytokine production [GO:0001817]; regulates GO:0032601